regulation of D-glucose transmembrane transport [GO:0010827] (biological process) Also known as: regulation of glucose transmembrane transport, regulation of glucose transport Relationships: is a type of regulation of transmembrane transport [GO:0034762]; regulates D-glucose transmembrane transport [GO:1904659] Definition: Any process that modulates the frequency, rate or extent of glucose transport across a membrane. Glucose transport is the directed movement of the hexose monosaccharide glucose into, out of or within a cell, or between cells, by means of some agent such as a transporter or pore. Sources: GOC:dph, GOC:tb Subtypes: positive regulation of D-glucose transmembrane transport [GO:0010828], negative regulation of D-glucose transmembrane transport [GO:0010829], regulation of D-glucose import [GO:0046324]